{
  "gene": "UniProtKB:O43914",
  "term_id": "GO:1904151",
  "gene_symbol": "TYROBP",
  "term_label": "positive regulation of microglial cell mediated cytotoxicity",
  "gene_name": "TYRO protein tyrosine kinase-binding protein"
}